L-histidine import across plasma membrane [GO:1903810] (biological process) Also known as: L-histidine import, histidine import, L-histidine import into cell References: PMID:23895341 Sources: GOC:TermGenie, GO_REF:0000075 Definition: The directed movement of L-histidine from outside of a cell, across the plasma membrane and into the cytosol. Relationships: is a type of L-histidine transmembrane transport [GO:0089709]; is a type of amino acid import across plasma membrane [GO:0089718]